calcium channel activity [GO:0005262] (molecular function) Subtypes: GO:0005245, stretch-activated, monoatomic cation-selective, calcium channel activity [GO:0015275], store-operated calcium channel activity [GO:0015279], GO:0099604 Regulation: regulated by GO:0005246; negatively regulated by calcium channel inhibitor activity [GO:0019855] Sources: GOC:mtg_transport, GOC:pr, ISBN:0815340729 Definition: Enables the energy-independent facilitated diffusion of a calcium ion through a transmembrane aqueous pore or channel. Relationships: is a type of monoatomic cation channel activity [GO:0005261]; is a type of calcium ion transmembrane transporter activity [GO:0015085]